allantoate deiminase activity [GO:0047652] (molecular function) Also known as: allantoate amidinohydrolase (decarboxylating), allantoate amidohydrolase activity Relationships: is a type of GO:0016813 Definition: Catalysis of the reaction: allantoate + H2O + H+ = CO2 + NH3 + ureidoglycine. Sources: EC:3.5.3.9, MetaCyc:ALLANTOATE-DEIMINASE-RXN